membrane fission [GO:0090148] (biological process) Definition: A process that is carried out at the cellular level which results in the separation of a single continuous membrane into two membranes. Sources: GOC:ascb_2009, GOC:dph, GOC:tb Also known as: membrane scission Relationships: is a type of membrane organization [GO:0061024] Subtypes: GO:0090149, vesicle scission [GO:0099050]